{
  "term_label": "RNA polymerase II transcription regulatory region sequence-specific DNA binding",
  "gene": "UniProtKB:Q9H7X3",
  "term_id": "GO:0000977",
  "gene_symbol": "ZNF696",
  "gene_name": "Zinc finger protein 696"
}